{
  "term_id": "UNKNOWN:0002",
  "term_label": "Unknown biological process",
  "gene_name": "Transmembrane protein 191A",
  "gene": "UniProtKB:Q9H0A3",
  "gene_symbol": "TMEM191A"
}